{
  "gene_symbol": "PTGER4",
  "gene_name": "Prostaglandin E2 receptor EP4 subtype",
  "term_label": "plasma membrane",
  "gene": "UniProtKB:P35408",
  "term_id": "GO:0005886"
}